{
  "term_id": "GO:0017134",
  "gene": "UniProtKB:O43427",
  "term_label": "fibroblast growth factor binding",
  "gene_symbol": "FIBP",
  "gene_name": "Acidic fibroblast growth factor intracellular-binding protein"
}